{
  "term_id": "GO:0031901",
  "gene": "UniProtKB:Q9HCC9",
  "term_label": "early endosome membrane",
  "gene_name": "Lateral signaling target protein 2 homolog",
  "gene_symbol": "ZFYVE28"
}